{
  "term_label": "Unknown cellular component",
  "term_id": "UNKNOWN:0003",
  "gene_symbol": "LGALS4",
  "gene": "UniProtKB:P56470",
  "gene_name": "Galectin-4"
}